{
  "term_id": "UNKNOWN:0001",
  "gene_name": "Collagen alpha-3(VI) chain",
  "gene": "UniProtKB:P12111",
  "term_label": "Unknown molecular function",
  "gene_symbol": "COL6A3"
}